{
  "gene_symbol": "PF4",
  "gene_name": "Platelet factor 4",
  "term_label": "extracellular space",
  "gene": "UniProtKB:P02776",
  "term_id": "GO:0005615"
}